{
  "gene_symbol": "DSEL",
  "term_id": "UNKNOWN:0003",
  "gene": "UniProtKB:Q8IZU8",
  "gene_name": "Dermatan-sulfate epimerase-like protein",
  "term_label": "Unknown cellular component"
}